negative regulation of lamellipodium morphogenesis [GO:2000393] (biological process) Sources: GOC:BHF, GOC:mah Also known as: negative regulation of lamellipodium organization Relationships: is a type of negative regulation of developmental process [GO:0051093]; is a type of negative regulation of lamellipodium organization [GO:1902744]; is a type of regulation of lamellipodium morphogenesis [GO:2000392]; negatively regulates lamellipodium morphogenesis [GO:0072673] Definition: Any process that stops, prevents or reduces the frequency, rate or extent of lamellipodium morphogenesis.